{
  "gene_symbol": "CERS6",
  "term_label": "endoplasmic reticulum",
  "term_id": "GO:0005783",
  "gene": "UniProtKB:Q6ZMG9",
  "gene_name": "Ceramide synthase 6"
}